{
  "gene_name": "Olfactory receptor 5I1",
  "gene_symbol": "OR5I1",
  "term_label": "olfactory receptor activity",
  "gene": "UniProtKB:Q13606",
  "term_id": "GO:0004984"
}